cargo adaptor activity [GO:0140312] (molecular function) References: PMID:25795254 Definition: Binding directly to the structural scaffolding elements of a vesicle coat (such as clathrin or COPII), and bridging the membrane, cargo receptor, and membrane deformation machinery. Subtypes: GO:0035615 Also known as: endocytic adaptor activity Relationships: is_a protein-macromolecule adaptor activity [GO:0030674]; is part of vesicle-mediated transport [GO:0016192]